mitochondrial degradosome [GO:0045025] (cellular component) References: PMID:10397341, PMID:9829834 Also known as: mtEXO Definition: A mitochondrial protein complex with 3' to 5' exoribonuclease activity that participates in intron-independent turnover and processing of mitochondrial transcripts. In humans, the mitochondrial degradosome is a pentameric complex, and in yeast it exists as a heterodimer. Relationships: is a type of GO:0098798; is a type of GO:1905354